{
  "term_id": "GO:0097190",
  "gene_symbol": "DAP",
  "gene_name": "Death-associated protein 1",
  "gene": "UniProtKB:P51397",
  "term_label": "apoptotic signaling pathway"
}